has_related_synonym [oboInOwl#hasRelatedSynonym]